extrachromosomal rDNA circle [GO:0005728] (cellular component) Definition: Circular DNA molecules encoding ribosomal RNA that are replicated independently of chromosomal replication. These molecules originate in the chromosome but are excised and circularized, often by intramolecular homologous recombination between direct tandem repeats. Also known as: extrachromosomal ribosomal DNA circle Relationships: is a type of extrachromosomal circular DNA [GO:0005727] References: PMID:12044934 Sources: GOC:mah